{
  "gene": "UniProtKB:Q9H7S9",
  "term_id": "GO:0045892",
  "gene_symbol": "ZNF703",
  "gene_name": "Zinc finger protein 703",
  "term_label": "negative regulation of DNA-templated transcription"
}